{
  "gene_symbol": "SFT2D2",
  "term_label": "Unknown molecular function",
  "term_id": "UNKNOWN:0001",
  "gene_name": "Vesicle transport protein SFT2B",
  "gene": "UniProtKB:O95562"
}